5'-deoxyribose-5-phosphate lyase activity [GO:0051575] (molecular function) Relationships: is a type of GO:0016835; is a type of catalytic activity, acting on DNA [GO:0140097] References: PMID:11251121, PMID:16120966, PMID:9614142 Sources: RHEA:76255 Also known as: dRP lyase activity, dRPase activity, 5'-deoxyribose phosphate activity Definition: Catalysis of the reaction: a 5'-end 2'-deoxyribose-2'-deoxyribonucleotide-DNA = (2E,4S)-4-hydroxypenten-2-al-5-phosphate + a 5'-end 5'-phospho-2'-deoxyribonucleoside-DNA + H+.